{
  "term_label": "interleukin-17 receptor activity",
  "term_id": "GO:0030368",
  "gene_name": "Interleukin-17 receptor C",
  "gene_symbol": "IL17RC",
  "gene": "UniProtKB:Q8NAC3"
}